{
  "gene_symbol": "COX7A1",
  "term_label": "oxidative phosphorylation",
  "term_id": "GO:0006119",
  "gene": "UniProtKB:P24310",
  "gene_name": "Cytochrome c oxidase subunit 7A1, mitochondrial"
}